{
  "gene_name": "Paired box protein Pax-4",
  "gene": "UniProtKB:O43316",
  "term_id": "GO:0007423",
  "term_label": "sensory organ development",
  "gene_symbol": "PAX4"
}